microtubule cytoskeleton [GO:0015630] (cellular component) Sources: GOC:jl, ISBN:0395825172 Relationships: is a type of cytoskeleton [GO:0005856] Definition: The part of the cytoskeleton (the internal framework of a cell) composed of microtubules and associated proteins.